{
  "term_id": "GO:0005615",
  "gene": "UniProtKB:P06276",
  "term_label": "extracellular space",
  "gene_name": "Cholinesterase",
  "gene_symbol": "BCHE"
}